{
  "term_label": "GTPase activator activity",
  "gene": "UniProtKB:Q8TDY4",
  "gene_name": "Arf-GAP with SH3 domain, ANK repeat and PH domain-containing protein 3",
  "gene_symbol": "ASAP3",
  "term_id": "GO:0005096"
}